{
  "gene_name": "ZZ-type zinc finger-containing protein 3",
  "term_id": "UNKNOWN:0002",
  "term_label": "Unknown biological process",
  "gene": "UniProtKB:Q8IYH5",
  "gene_symbol": "ZZZ3"
}